{
  "gene_symbol": "PDIA3",
  "term_label": "cell surface",
  "term_id": "GO:0009986",
  "gene": "UniProtKB:P30101",
  "gene_name": "Protein disulfide-isomerase A3"
}